{
  "gene_name": "Endothelin-converting enzyme 1",
  "term_id": "GO:0016486",
  "gene_symbol": "ECE1",
  "term_label": "peptide hormone processing",
  "gene": "UniProtKB:P42892"
}